regulation of icosanoid secretion [GO:0032303] (biological process) Sources: GOC:mah Definition: Any process that modulates the frequency, rate or extent of the controlled release of an icosanoid from a cell. Also known as: regulation of eicosanoid secretion Subtypes: negative regulation of icosanoid secretion [GO:0032304], positive regulation of icosanoid secretion [GO:0032305], regulation of prostaglandin secretion [GO:0032306], GO:0090237 Relationships: is a type of regulation of secretion [GO:0051046]; is a type of regulation of fatty acid transport [GO:2000191]; RO_0002211 icosanoid secretion [GO:0032309]